positive regulation of leukocyte adhesion to vascular endothelial cell [GO:1904996] (biological process) References: PMID:23897866 Sources: GOC:BHF, GOC:BHF_miRNA, GOC:TermGenie, GOC:bc, GO_REF:0000058 Subtypes: positive regulation of leukocyte tethering or rolling [GO:1903238], GO:1904999 Relationships: is a type of GO:1903039; is a type of regulation of leukocyte adhesion to vascular endothelial cell [GO:1904994]; positively regulates leukocyte adhesion to vascular endothelial cell [GO:0061756] Also known as: up regulation of leukocyte adhesion to vascular endothelial cell, up-regulation of leukocyte adhesion to vascular endothelial cell, upregulation of leukocyte adhesion to vascular endothelial cell, activation of leukocyte adhesion to vascular endothelial cell Definition: Any process that activates or increases the frequency, rate or extent of leukocyte adhesion to vascular endothelial cell.